non-proteinogenic amino acid metabolic process [GO:0170041] (biological process) Also known as: non-proteinogenic amino acid metabolism Subtypes: citrulline metabolic process [GO:0000052], argininosuccinate metabolic process [GO:0000053], GO:0006591, GO:0009448, peptidyl-proline hydroxylation to 3-hydroxy-L-proline [GO:0018400], peptidyl-proline hydroxylation to 4-hydroxy-L-proline [GO:0018401], 1-aminocyclopropane-1-carboxylate metabolic process [GO:0018871], L-methionine biosynthetic process from L-homoserine via cystathionine [GO:0019279], GO:0019280, L-methionine biosynthetic process from L-homoserine via O-phospho-L-homoserine and cystathionine [GO:0019283], beta-alanine metabolic process [GO:0019482], GO:0046416, S-adenosylhomocysteine metabolic process [GO:0046498], GO:0046516, GO:0050667, kynurenine metabolic process [GO:0070189], non-proteinogenic amino acid biosynthetic process [GO:0170043], non-proteinogenic amino acid catabolic process [GO:0170044], GO:1901052, L-dopa metabolic process [GO:1903184] Sources: GOC:ew Definition: The chemical reactions and pathways involving non-proteingenic amino acids. Relationships: is a type of amino acid metabolic process [GO:0006520]; is a type of GO:0019752